{
  "term_label": "flavin adenine dinucleotide binding",
  "gene": "UniProtKB:P16435",
  "gene_name": "NADPH--cytochrome P450 reductase",
  "gene_symbol": "POR",
  "term_id": "GO:0050660"
}